mesothelial-mesenchymal cell signaling involved in early lung development [GO:0061142] (biological process) Sources: GOC:dph Relationships: is a type of GO:0060495 Definition: Any process that mediates the transfer of information from a mesothelial cell to an epithelial cell and contributes to the development of the lung. Also known as: mesothelial-mesenchymal cell signalling involved in early lung development